{
  "gene_name": "Cap-specific mRNA (nucleoside-2'-O-)-methyltransferase 2",
  "gene": "UniProtKB:Q8IYT2",
  "term_label": "methyltransferase cap1 activity",
  "term_id": "GO:0004483",
  "gene_symbol": "CMTR2"
}